raffinose biosynthetic process [GO:0033529] (biological process) Regulation: regulated by regulation of raffinose biosynthetic process [GO:1900091]; negatively regulated by GO:1900092; positively regulated by positive regulation of raffinose biosynthetic process [GO:1900093] Relationships: is a type of raffinose family oligosaccharide biosynthetic process [GO:0010325]; is a type of raffinose metabolic process [GO:0033530] Sources: GOC:mah Also known as: raffinose anabolism, raffinose biosynthesis, raffinose formation, raffinose synthesis Definition: The chemical reactions and pathways resulting in the formation of raffinose, the trisaccharide beta-D-fructofuranosyl alpha-D-galactopyranosyl-(1->6)-alpha-D-glucopyranoside.